syncytial embryo cellularization [GO:0110069] (biological process) References: PMID:27226317 Sources: GOC:ha Definition: The separation of a syncytial embryo into individual cells. Relationships: is_a cellularization [GO:0007349]; is a type of GO:0051301; is part of embryo development [GO:0009790]